seminal vesicle epithelium development [GO:0061108] (biological process) Sources: GOC:dph Relationships: is a type of developmental process involved in reproduction [GO:0003006]; is a type of tube development [GO:0035295]; is a type of epithelium development [GO:0060429]; is part of GO:0061107 Definition: The progression of the seminal vesicle epithelium over time, from its formation to the mature structure.